{
  "gene_name": "Glutathione hydrolase 1 proenzyme",
  "gene_symbol": "GGT1",
  "term_label": "regulation of inflammatory response",
  "gene": "UniProtKB:P19440",
  "term_id": "GO:0050727"
}